{
  "gene": "UniProtKB:Q96JY6",
  "term_label": "adherens junction",
  "term_id": "GO:0005912",
  "gene_name": "PDZ and LIM domain protein 2",
  "gene_symbol": "PDLIM2"
}